positive regulation of synaptic assembly at neuromuscular junction [GO:0045887] (biological process) Relationships: is a type of regulation of synaptic assembly at neuromuscular junction [GO:0008582]; is a type of positive regulation of developmental growth [GO:0048639]; is a type of GO:0051965; is a type of GO:1904398; positively regulates synaptic assembly at neuromuscular junction [GO:0051124] Definition: Any process that activates or increases the frequency, rate or extent of synaptic assembly at neuromuscular junction. Also known as: up regulation of synaptic growth at neuromuscular junction, up-regulation of synaptic growth at neuromuscular junction, upregulation of synaptic growth at neuromuscular junction, activation of synaptic growth at neuromuscular junction, stimulation of synaptic growth at neuromuscular junction, positive regulation of synaptic growth at neuromuscular junction Sources: GOC:go_curators